{
  "term_label": "cytoplasm",
  "gene_name": "Proto-oncogene vav",
  "gene": "UniProtKB:P15498",
  "gene_symbol": "VAV1",
  "term_id": "GO:0005737"
}